{
  "gene_symbol": "PER1",
  "gene_name": "Period circadian protein homolog 1",
  "term_label": "circadian regulation of gene expression",
  "term_id": "GO:0032922",
  "gene": "UniProtKB:O15534"
}